glycosaminoglycan catabolic process [GO:0006027] (biological process) Also known as: glycosaminoglycan breakdown, glycosaminoglycan catabolism, glycosaminoglycan degradation Definition: The chemical reactions and pathways resulting in the breakdown of glycosaminoglycans, any one of a group of linear polysaccharides composed of repeating disaccharide units. Relationships: is a type of GO:0006026; is a type of glycosaminoglycan metabolic process [GO:0030203] Subtypes: peptidoglycan catabolic process [GO:0009253], hyaluronan catabolic process [GO:0030214] References: PMID:38500384